{
  "gene_name": "E3 ubiquitin-protein ligase MARCHF2",
  "term_id": "GO:0016567",
  "gene": "UniProtKB:Q9P0N8",
  "term_label": "protein ubiquitination",
  "gene_symbol": "MARCHF2"
}